glycerol-3-phosphate 2-O-acyltransferase activity [GO:0090447] (molecular function) Definition: Catalysis of the reaction: an acyl-CoA + sn-glycerol 3-phosphate = CoA + a 2-acyl-sn-glycerol 3-phosphate. Sources: RHEA:33559 Relationships: is a type of O-acyltransferase activity [GO:0008374]